gap junction channel activity involved in bundle of His cell-Purkinje myocyte electrical coupling [GO:0086078] (molecular function) Sources: GOC:BHF, GOC:mtg_cardiac_conduct_nov11 Relationships: is a type of gap junction channel activity involved in cardiac conduction electrical coupling [GO:0086075]; is part of GO:0086054 Definition: A wide pore channel activity that enables a direct cytoplasmic connection from a bundle of His cell to a Purkinje myocyte. The gap junction passes electrical signals between the cells contributing to cardiac conduction.